archaetidylserine synthase activity [GO:0043761] (molecular function) Definition: Catalysis of the reaction: CDP-digeranylgeranylglycerol + L-serine = archaetidylserine + CMP. References: PMID:12562787 Also known as: CDP-2,3-di-O-geranylgeranyl-sn-glycerol inositol 1-archaetidyltransferase activity, CDP-2,3-di-O-geranylgeranyl-sn-glycerol:l-serine O-archaetidyltransferase activity Relationships: is a type of GO:0016780